negative regulation of protein metabolic process [GO:0051248] (biological process) Definition: Any process that stops, prevents, or reduces the frequency, rate or extent of chemical reactions and pathways involving a protein. Sources: GOC:ai Also known as: down regulation of cellular protein metabolic process, down regulation of protein metabolic process, down-regulation of cellular protein metabolic process, down-regulation of protein metabolic process, downregulation of cellular protein metabolic process, downregulation of protein metabolic process, negative regulation of cellular protein metabolic process, negative regulation of cellular protein metabolism, negative regulation of protein metabolism, inhibition of cellular protein metabolic process, inhibition of protein metabolic process Relationships: is a type of negative regulation of macromolecule metabolic process [GO:0010605]; is_a regulation of protein metabolic process [GO:0051246]; negatively regulates protein metabolic process [GO:0019538] Subtypes: GO:0017148, negative regulation of protein modification process [GO:0031400], GO:0032685, negative regulation of hepatocyte growth factor production [GO:0032686], negative regulation of lymphotoxin A production [GO:0032721], GO:0042177, negative regulation of proteolysis [GO:0045861], negative regulation of hemoglobin biosynthetic process [GO:0046986], GO:0050748, GO:1902992, negative regulation of glycoprotein metabolic process [GO:1903019], negative regulation of protein maturation [GO:1903318], GO:1905907